regulation of tensidol B biosynthetic process [GO:1900710] (biological process) Sources: GOC:TermGenie, GOC:di Also known as: regulation of tensidol B anabolism, regulation of tensidol B biosynthesis, regulation of tensidol B formation, regulation of tensidol B synthesis Subtypes: negative regulation of tensidol B biosynthetic process [GO:1900711], positive regulation of tensidol B biosynthetic process [GO:1900712] Definition: Any process that modulates the frequency, rate or extent of tensidol B biosynthetic process. Relationships: is a type of regulation of ketone biosynthetic process [GO:0010566]; is a type of regulation of amide metabolic process [GO:0034248]; is a type of regulation of secondary metabolite biosynthetic process [GO:1900376]; RO_0002211 GO:1900608